{
  "term_id": "GO:0006955",
  "gene_name": "Immunoglobulin kappa variable 3D-11",
  "term_label": "immune response",
  "gene": "UniProtKB:A0A0A0MRZ8",
  "gene_symbol": "IGKV3D-11"
}